{
  "gene": "UniProtKB:P45974",
  "gene_symbol": "USP5",
  "term_label": "cysteine-type deubiquitinase activity",
  "gene_name": "Ubiquitin carboxyl-terminal hydrolase 5",
  "term_id": "GO:0004843"
}